{
  "term_id": "GO:0051014",
  "term_label": "actin filament severing",
  "gene": "UniProtKB:P09327",
  "gene_name": "Villin-1",
  "gene_symbol": "VIL1"
}